succinyltransferase activity [GO:0016748] (molecular function) Definition: Catalysis of the transfer of a succinyl (3-carboxypropanoyl) group to an acceptor molecule. Relationships: is a type of acyltransferase activity, transferring groups other than amino-acyl groups [GO:0016747] Sources: GOC:ai Subtypes: N-succinyltransferase activity [GO:0016749], GO:0016750, GO:0016751